{
  "gene": "UniProtKB:P23109",
  "term_label": "cytosol",
  "gene_name": "AMP deaminase 1",
  "gene_symbol": "AMPD1",
  "term_id": "GO:0005829"
}